glycolipid floppase activity [GO:0034202] (molecular function) Relationships: is a type of floppase activity [GO:0140328]; BFO_0000050 glycolipid translocation [GO:0034203] Also known as: ATP-dependent intramembrane glycolipid transporter activity, ATPase-coupled intramembrane glycolipid transporter activity, glycolipid-translocating activity, glycolipid floppase activity (cytosolic to exoplasmic leaflet), M5GN2-PP-Dol flippase activity, Man(5)GlcNAc(2)-PP-dolichol translocator, Man5GlcNac2-PP-Dol ER flippase activity References: PMID:11807558 Sources: GOC:krc Definition: Catalysis of the movement of a glycolipid from the cytosolic to the exoplasmic leaflet of a membrane, using energy from the hydrolysis of ATP.